fatty acid catabolic process [GO:0009062] (biological process) Subtypes: fatty acid alpha-oxidation [GO:0001561], GO:0006635, short-chain fatty acid catabolic process [GO:0019626], lipoate catabolic process [GO:0032323], GO:0042758, very long-chain fatty acid catabolic process [GO:0042760], butyryl-CoA catabolic process [GO:0044580], medium-chain fatty acid catabolic process [GO:0051793], GO:1903965, anaerobic fatty acid catabolic process [GO:1990486] Sources: GOC:go_curators Relationships: is a type of fatty acid metabolic process [GO:0006631]; is a type of lipid catabolic process [GO:0016042]; is a type of monocarboxylic acid catabolic process [GO:0072329] Definition: The chemical reactions and pathways resulting in the breakdown of a fatty acid, any of the aliphatic monocarboxylic acids that can be liberated by hydrolysis from naturally occurring fats and oils. Fatty acids are predominantly straight-chain acids of 4 to 24 carbon atoms, which may be saturated or unsaturated; branched fatty acids and hydroxy fatty acids also occur, and very long chain acids of over 30 carbons are found in waxes. Also known as: fatty acid breakdown, fatty acid catabolism, fatty acid degradation